{
  "gene": "UniProtKB:Q0VDF9",
  "gene_symbol": "HSPA14",
  "gene_name": "Heat shock 70 kDa protein 14",
  "term_label": "protein refolding",
  "term_id": "GO:0042026"
}